{
  "gene_symbol": "CHN1",
  "gene_name": "N-chimaerin",
  "gene": "UniProtKB:P15882",
  "term_label": "ephrin receptor signaling pathway",
  "term_id": "GO:0048013"
}